DNA negative supercoiling activity [GO:0034335] (molecular function) Relationships: is a type of GO:0003918 Also known as: DNA gyrase activity, DNA-gyrase activity Note: Note that this term was reinstated from obsolete. Definition: Catalytic introduction of negative supercoils into a DNA molecule or region thereof. In bacteria, negative supercoils are only introduced by DNA gyrase, a type II topoisomerase, but not all DNA gyrases are capable of introducing supercoils. In bacteria, the level of supercoiling varies widely between species and has been characterized properly in only a handful of organisms. The best characterized enzyme, from E.coli, is exceptionally proficient at supercoiling and this ability is not representative of all bacteria. Sources: GOC:bhm, GOC:krc, GOC:mah, WikiPedia:DNA_gyrase